{
  "term_label": "regulation of protein localization",
  "gene_symbol": "TMEM231",
  "gene_name": "Transmembrane protein 231",
  "term_id": "GO:0032880",
  "gene": "UniProtKB:Q9H6L2"
}